negative regulation of amyloid-beta formation [GO:1902430] (biological process) Relationships: is a type of negative regulation of amide metabolic process [GO:0034249]; is a type of GO:1902003; is a type of GO:1902992; negatively regulates amyloid-beta formation [GO:0034205] Also known as: down regulation of beta-amyloid formation, down-regulation of beta-amyloid formation, downregulation of beta-amyloid formation, negative regulation of beta-amyloid formation, inhibition of beta-amyloid formation References: PMID:22992957 Sources: GOC:TermGenie, GOC:hjd Definition: Any process that stops, prevents or reduces the frequency, rate or extent of amyloid-beta formation.